{
  "gene_symbol": "PIK3C2B",
  "gene_name": "Phosphatidylinositol 4-phosphate 3-kinase C2 domain-containing subunit beta",
  "term_id": "GO:0036092",
  "gene": "UniProtKB:O00750",
  "term_label": "phosphatidylinositol-3-phosphate biosynthetic process"
}